rhombomere 4 formation [GO:0021663] (BP) Sources: GOC:cls, GOC:curators, GOC:dgh, GOC:dph, GOC:jid Definition: The process that gives rise to rhombomere 4. This process pertains to the initial formation of a structure from unspecified parts. Rhombomeres are transverse segments of the developing rhombencephalon. Rhombomeres are lineage restricted, express different genes from one another, and adopt different developmental fates. Rhombomeres are numbered in anterior to posterior order. Relationships: is_a rhombomere formation [GO:0021594]; is part of rhombomere 4 morphogenesis [GO:0021661]